{
  "term_id": "GO:0004331",
  "gene": "UniProtKB:P16118",
  "gene_name": "6-phosphofructo-2-kinase_fructose-2,6-bisphosphatase 1",
  "term_label": "fructose-2,6-bisphosphate 2-phosphatase activity",
  "gene_symbol": "PFKFB1"
}